{
  "gene_symbol": "GLMP",
  "term_label": "Unknown molecular function",
  "gene_name": "Glycosylated lysosomal membrane protein",
  "term_id": "UNKNOWN:0001",
  "gene": "UniProtKB:Q8WWB7"
}